{
  "gene_symbol": "PLP2",
  "gene": "UniProtKB:Q04941",
  "term_label": "Unknown biological process",
  "term_id": "UNKNOWN:0002",
  "gene_name": "Proteolipid protein 2"
}